{
  "gene_name": "Olfactory receptor 2T8",
  "gene": "UniProtKB:A6NH00",
  "term_id": "GO:0004984",
  "term_label": "olfactory receptor activity",
  "gene_symbol": "OR2T8"
}